{
  "gene": "UniProtKB:Q8WWR8",
  "term_label": "oligosaccharide catabolic process",
  "gene_symbol": "NEU4",
  "gene_name": "Sialidase-4",
  "term_id": "GO:0009313"
}